{
  "term_id": "UNKNOWN:0003",
  "gene_symbol": "C2orf83",
  "gene": "UniProtKB:Q53S99",
  "gene_name": "Folate transporter-like protein C2orf83",
  "term_label": "Unknown cellular component"
}